{
  "gene_symbol": "A0A1W2PQF6",
  "term_label": "immune response-inhibiting cell surface receptor signaling pathway",
  "term_id": "GO:0002767",
  "gene": "UniProtKB:A0A1W2PQF6",
  "gene_name": "Immunoglobulin subtype domain-containing protein"
}